{
  "gene": "UniProtKB:Q9H6R3",
  "gene_name": "Acyl-CoA synthetase short-chain family member 3, mitochondrial",
  "term_id": "GO:0050218",
  "term_label": "propionate-CoA ligase activity",
  "gene_symbol": "ACSS3"
}